{
  "gene_symbol": "APOL2",
  "gene_name": "Apolipoprotein L2",
  "term_id": "UNKNOWN:0003",
  "term_label": "Unknown cellular component",
  "gene": "UniProtKB:Q9BQE5"
}